mechanosensitive monoatomic ion channel activity [GO:0008381] (molecular function) Definition: Enables the transmembrane transfer of an monoatomic ion by a channel that opens in response to a mechanical stress. Sources: GOC:mtg_transport, ISBN:0815340729 Also known as: mechanosensitive ion channel activity, mechanically gated channel activity, mechanically-gated channel activity, mechanically-gated ion channel activity Relationships: is a type of monoatomic ion channel activity [GO:0005216]; is a type of gated channel activity [GO:0022836] Subtypes: cyclic nucleotide-gated mechanosensitive monoatomic ion channel activity [GO:0043854], mechanosensitive monoatomic cation channel activity [GO:0140135]